{
  "gene_name": "Myosin-10",
  "gene_symbol": "MYH10",
  "term_label": "microfilament motor activity",
  "gene": "UniProtKB:P35580",
  "term_id": "GO:0000146"
}